dendritic transport of mitochondrion [GO:0098939] (biological process) Sources: GOC:ai Relationships: is a type of mitochondrion transport along microtubule [GO:0047497]; is a type of dendritic transport [GO:0098935]; occurs in GO:0032839 Definition: The directed movement of mitochondria along microtubules in nerve cell dendrites. Subtypes: retrograde dendritic transport of mitochondrion [GO:0098959], GO:0098972